{
  "gene_symbol": "SPPL2C",
  "term_id": "GO:0098554",
  "gene_name": "Signal peptide peptidase-like 2C",
  "term_label": "cytoplasmic side of endoplasmic reticulum membrane",
  "gene": "UniProtKB:Q8IUH8"
}